GDP-galactose:myoinositol-1-phosphate guanylyltransferase activity [GO:0010473] (molecular function) References: PMID:17485667 Relationships: is a type of GO:0070568 Definition: Catalysis of the reaction: GDP-L-galactose + myo-inositol 1-phosphate = alpha-L-galactose-1-phosphate + GDP-myoinositol.